negative regulation of DNA metabolic process [GO:0051053] (biological process) Also known as: down regulation of DNA metabolic process, down-regulation of DNA metabolic process, downregulation of DNA metabolic process, negative regulation of DNA metabolism, inhibition of DNA metabolic process Relationships: is a type of negative regulation of macromolecule metabolic process [GO:0010605]; is a type of negative regulation of nucleobase-containing compound metabolic process [GO:0045934]; is a type of GO:0051052; negatively regulates DNA metabolic process [GO:0006259] Definition: Any process that stops, prevents, or reduces the frequency, rate or extent of the chemical reactions and pathways involving DNA. Subtypes: GO:0008156, negative regulation of telomere maintenance [GO:0032205], negative regulation of DNA repair [GO:0045738], GO:0045910, negative regulation of mitotic recombination-dependent replication fork processing [GO:0120291], negative regulation of mitochondrial DNA metabolic process [GO:1901859], negative regulation of meiotic DNA double-strand break formation [GO:1903342], negative regulation of DNA catabolic process [GO:1903625], GO:1904430, negative regulation of DNA biosynthetic process [GO:2000279] Sources: GOC:ai